{
  "gene_symbol": "MFSD6",
  "term_id": "GO:0005886",
  "gene_name": "Major facilitator superfamily domain-containing protein 6",
  "term_label": "plasma membrane",
  "gene": "UniProtKB:Q6ZSS7"
}